{
  "term_label": "G protein-coupled receptor activity",
  "gene_symbol": "ADGRE2",
  "gene_name": "Adhesion G protein-coupled receptor E2",
  "term_id": "GO:0004930",
  "gene": "UniProtKB:Q9UHX3"
}